{
  "gene": "UniProtKB:Q9BTE6",
  "gene_name": "Alanyl-tRNA editing protein Aarsd1",
  "term_id": "GO:0002196",
  "gene_symbol": "AARSD1",
  "term_label": "Ser-tRNA(Ala) deacylase activity"
}